{
  "gene_name": "Ectonucleoside triphosphate diphosphohydrolase 8",
  "term_id": "GO:0009134",
  "gene": "UniProtKB:Q5MY95",
  "term_label": "nucleoside diphosphate catabolic process",
  "gene_symbol": "ENTPD8"
}